{
  "term_label": "Cajal body",
  "gene": "UniProtKB:P38432",
  "gene_symbol": "COIL",
  "gene_name": "Coilin",
  "term_id": "GO:0015030"
}